{
  "term_label": "cell surface",
  "term_id": "GO:0009986",
  "gene_name": "Leucine-rich repeat and fibronectin type-III domain-containing protein 3",
  "gene": "UniProtKB:Q9BTN0",
  "gene_symbol": "LRFN3"
}